{
  "gene": "UniProtKB:Q8TEL6",
  "term_id": "GO:0006511",
  "gene_name": "Short transient receptor potential channel 4-associated protein",
  "term_label": "ubiquitin-dependent protein catabolic process",
  "gene_symbol": "TRPC4AP"
}